{
  "gene_symbol": "FOCAD",
  "term_label": "Unknown cellular component",
  "gene_name": "Focadhesin",
  "term_id": "UNKNOWN:0003",
  "gene": "UniProtKB:Q5VW36"
}